{
  "term_label": "nuclear envelope",
  "gene_name": "Sperm-associated antigen 4 protein",
  "gene_symbol": "SPAG4",
  "term_id": "GO:0005635",
  "gene": "UniProtKB:Q9NPE6"
}